{
  "term_label": "phosphatidylserine binding",
  "gene": "UniProtKB:Q494U1",
  "gene_symbol": "PLEKHN1",
  "gene_name": "Pleckstrin homology domain-containing family N member 1",
  "term_id": "GO:0001786"
}